{
  "term_label": "Unknown biological process",
  "gene_name": "DNA-directed RNA polymerase III subunit RPC10",
  "term_id": "UNKNOWN:0002",
  "gene": "UniProtKB:Q9Y2Y1",
  "gene_symbol": "POLR3K"
}